{
  "term_id": "GO:0006627",
  "term_label": "protein processing involved in protein targeting to mitochondrion",
  "gene_symbol": "MIPEP",
  "gene": "UniProtKB:Q99797",
  "gene_name": "Mitochondrial intermediate peptidase"
}